NADH dehydrogenase complex [GO:0030964] (cellular component) Relationships: is a type of GO:0098796; is a type of oxidoreductase complex [GO:1990204] Subtypes: respiratory chain complex I [GO:0045271], GO:0071685 Sources: GOC:mah Note: Note that this term represents a location and not a function; the activity possessed by this complex is mentioned in the definition for the purpose of describing and distinguishing the complex. The function possessed by this complex is represented by the molecular function term 'NADH dehydrogenase (quinone) activity ; GO:0050136'. Definition: An integral membrane complex that possesses NADH oxidoreductase activity. The complex is one of the components of the electron transport chain. It catalyzes the transfer of a pair of electrons from NADH to a quinone. Also known as: NADH dehydrogenase complex (plastoquinone), NADH dehydrogenase complex (quinone), NADH dehydrogenase complex (ubiquinone), NADH:plastoquinone reductase complex, plastid NADH dehydrogenase complex (plastoquinone)